{
  "term_label": "cytoplasm",
  "gene_symbol": "FHOD3",
  "term_id": "GO:0005737",
  "gene": "UniProtKB:Q2V2M9",
  "gene_name": "FH1_FH2 domain-containing protein 3"
}